{
  "gene_name": "Platelet-derived growth factor D",
  "term_id": "GO:0008284",
  "term_label": "positive regulation of cell population proliferation",
  "gene_symbol": "PDGFD",
  "gene": "UniProtKB:Q9GZP0"
}